high-affinity L-histidine transmembrane transporter activity [GO:0005291] (molecular function) Also known as: high affinity L-histidine transmembrane transporter activity, high affinity histidine permease activity Relationships: is_a high-affinity basic amino acid transmembrane transporter activity [GO:0005287]; is a type of L-histidine transmembrane transporter activity [GO:0005290] Sources: GOC:mtg_transport Definition: Enables the transfer of L-histidine from one side of a membrane to the other. L-histidine is 2-amino-3-(1H-imidazol-4-yl)propanoic acid. In high-affinity transport the transporter is able to bind the solute even if it is only present at very low concentrations.